cellubrevin-VAMP4-syntaxin-16 complex [GO:0070065] (cellular component) Relationships: is_a SNARE complex [GO:0031201] Also known as: SNARE complex (Vamp3, Vamp4, Stx16), Vamp3-Vamp4-Stx16 complex References: PMID:11839770 Definition: A SNARE complex that contains cellubrevin (VAMP3), VAMP4, and syntaxin 16 (or orthologs thereof).